{
  "term_label": "heparosan-N-sulfate-glucuronate 5-epimerase activity",
  "gene": "UniProtKB:O94923",
  "gene_name": "D-glucuronyl C5-epimerase",
  "gene_symbol": "GLCE",
  "term_id": "GO:0047464"
}